{
  "gene_symbol": "PRAME",
  "term_label": "Cul2-RING ubiquitin ligase complex",
  "gene_name": "Melanoma antigen preferentially expressed in tumors",
  "term_id": "GO:0031462",
  "gene": "UniProtKB:P78395"
}